establishment or maintenance of polarity of follicular epithelium [GO:0016334] (biological process) Sources: GOC:bf, GOC:mah Definition: Any cellular process that results in the specification, formation or maintenance of a polarized follicular epithelial sheet. Relationships: is a type of establishment or maintenance of cell polarity [GO:0007163]; is part of GO:0016333 Subtypes: dorsal/ventral axis specification, ovarian follicular epithelium [GO:0008069], anterior/posterior axis specification, follicular epithelium [GO:0030714], GO:0042247, maintenance of polarity of follicular epithelium [GO:0042248]